{
  "gene": "UniProtKB:Q96A05",
  "term_id": "GO:0046961",
  "gene_symbol": "ATP6V1E2",
  "gene_name": "V-type proton ATPase subunit E 2",
  "term_label": "proton-transporting ATPase activity, rotational mechanism"
}